adenylate cyclase-inhibiting G protein-coupled receptor signaling pathway [GO:0007193] (biological process) Relationships: is a type of GO:0007188; has part adenylate cyclase inhibitor activity [GO:0010855] Definition: A G protein-coupled receptor signaling pathway in which the signal is transmitted via the inhibition of adenylyl cyclase activity and a subsequent decrease in the intracellular concentration of cyclic AMP (cAMP). Subtypes: adenylate cyclase-inhibiting dopamine receptor signaling pathway [GO:0007195], adenylate cyclase-inhibiting G protein-coupled glutamate receptor signaling pathway [GO:0007196], adenylate cyclase-inhibiting G protein-coupled acetylcholine receptor signaling pathway [GO:0007197], adenylate cyclase-inhibiting serotonin receptor signaling pathway [GO:0007198], adenylate cyclase-inhibiting opioid receptor signaling pathway [GO:0031635], adenylate cyclase-inhibiting adrenergic receptor signaling pathway [GO:0071881] Note: This term is intended to cover steps in a GPCR signaling pathway both upstream and downstream of adenylate-cyclase inhibition. Sources: GOC:dph, GOC:mah, GOC:signaling, GOC:tb, ISBN:0815316194 Also known as: G protein signaling, adenylate cyclase inhibiting pathway, G protein signaling, adenylyl cyclase inhibiting pathway, G protein signalling, adenylate cyclase inhibiting pathway, G protein signalling, adenylyl cyclase inhibiting pathway, G-protein signaling, adenylate cyclase inhibiting pathway, G-protein signaling, adenylyl cyclase inhibiting pathway, G-protein signalling, adenylate cyclase inhibiting pathway, G-protein signalling, adenylyl cyclase inhibiting pathway, GPCR signaling pathway via inhibition of adenylate cyclase activity, adenylate cyclase-inhibiting GPCR signaling pathway, inhibition of adenylate cyclase activity by G-protein signaling pathway